{
  "term_id": "GO:2000096",
  "term_label": "positive regulation of Wnt signaling pathway, planar cell polarity pathway",
  "gene": "UniProtKB:Q9H4M7",
  "gene_symbol": "PLEKHA4",
  "gene_name": "Pleckstrin homology domain-containing family A member 4"
}